{
  "gene_symbol": "PCIF1",
  "term_id": "UNKNOWN:0001",
  "gene": "UniProtKB:Q9H4Z3",
  "term_label": "Unknown molecular function",
  "gene_name": "mRNA (2'-O-methyladenosine-N(6)-)-methyltransferase"
}